protein transport along microtubule to cell tip [GO:0099117] (biological process) Definition: The movement of a protein along a microtubule to the cell-tip, mediated by motor proteins. References: PMID:15177031 Relationships: is a type of protein transport along microtubule [GO:0098840]; is a type of protein localization to cell tip [GO:1990151]